neural fold elevation formation [GO:0021502] (biological process) References: PMID:15806586 Sources: GOC:cls, GOC:dgh, GOC:dph, GOC:jid, GO_REF:0000021 Definition: The process in which the lateral borders of the neural plate begin to migrate upwards to form the neural folds, caused by the proliferation of the underlying mesoderm. Relationships: is a type of GO:0048646; is part of GO:0001842